{
  "term_label": "cone photoreceptor outer segment",
  "gene_symbol": "GUCA1A",
  "gene": "UniProtKB:P43080",
  "term_id": "GO:0120199",
  "gene_name": "Guanylyl cyclase-activating protein 1"
}